{
  "gene": "UniProtKB:Q13443",
  "gene_name": "Disintegrin and metalloproteinase domain-containing protein 9",
  "term_label": "membrane protein ectodomain proteolysis",
  "gene_symbol": "ADAM9",
  "term_id": "GO:0006509"
}